{
  "gene_symbol": "DNAJC1",
  "gene_name": "DnaJ homolog subfamily C member 1",
  "term_id": "GO:0012505",
  "term_label": "endomembrane system",
  "gene": "UniProtKB:Q96KC8"
}